{
  "gene_symbol": "F2R",
  "term_id": "GO:0007200",
  "gene": "UniProtKB:P25116",
  "term_label": "phospholipase C-activating G protein-coupled receptor signaling pathway",
  "gene_name": "Proteinase-activated receptor 1"
}